{
  "term_id": "UNKNOWN:0003",
  "term_label": "Unknown cellular component",
  "gene_symbol": "C1orf115",
  "gene": "UniProtKB:Q9H7X2",
  "gene_name": "Required for drug-induced death protein 1"
}